{
  "gene_symbol": "ARHGEF40",
  "gene_name": "Rho guanine nucleotide exchange factor 40",
  "gene": "UniProtKB:Q8TER5",
  "term_id": "GO:0005737",
  "term_label": "cytoplasm"
}